intestinal D-glucose absorption [GO:0001951] (biological process) Relationships: is a type of intestinal hexose absorption [GO:0106001] Regulation: regulated by regulation of intestinal D-glucose absorption [GO:1903985] Definition: Uptake of D-glucose into the blood by absorption from the small intestine. References: PMID:5601832 Sources: GOC:mgi_curators